adult behavior [GO:0030534] (BP) Also known as: adult behavioral response to stimulus, adult behaviour, adult behavioural response to stimulus Note: See also the biological process term 'behavior ; GO:0007610'. Subtypes: adult feeding behavior [GO:0008343], adult locomotory behavior [GO:0008344], GO:0035095, behavioral response to cocaine [GO:0048148], behavioral response to ethanol [GO:0048149], GO:0048150 Definition: Behavior in a fully developed and mature organism. Relationships: is a type of GO:0007610 Sources: GOC:mah, ISBN:0877797099